{
  "gene_symbol": "KSR2",
  "gene_name": "Kinase suppressor of Ras 2",
  "gene": "UniProtKB:Q6VAB6",
  "term_id": "GO:0005829",
  "term_label": "cytosol"
}